{
  "gene": "UniProtKB:P61020",
  "term_label": "endocytic vesicle",
  "term_id": "GO:0030139",
  "gene_symbol": "RAB5B",
  "gene_name": "Ras-related protein Rab-5B"
}